forebrain morphogenesis [GO:0048853] (biological process) Also known as: prosencephalon morphogenesis Sources: GOC:cvs, GOC:dgh, GOC:dph, GOC:jid Definition: The process in which the anatomical structures of the forebrain are generated and organized. The forebrain is the anterior of the three primary divisions of the developing chordate brain or the corresponding part of the adult brain (in vertebrates, includes especially the cerebral hemispheres, the thalamus, and the hypothalamus and especially in higher vertebrates is the main control center for sensory and associative information processing, visceral functions, and voluntary motor functions). Relationships: is a type of anatomical structure morphogenesis [GO:0009653]; is part of forebrain development [GO:0030900]; is part of brain morphogenesis [GO:0048854]